{
  "term_label": "GTPase activity",
  "term_id": "GO:0003924",
  "gene": "UniProtKB:Q7L523",
  "gene_name": "Ras-related GTP-binding protein A",
  "gene_symbol": "RRAGA"
}